{
  "gene_name": "Testisin",
  "term_id": "GO:0006508",
  "gene": "UniProtKB:Q9Y6M0",
  "term_label": "proteolysis",
  "gene_symbol": "PRSS21"
}